{
  "gene": "UniProtKB:P10909",
  "term_label": "positive regulation of proteasomal ubiquitin-dependent protein catabolic process",
  "gene_symbol": "CLU",
  "term_id": "GO:0032436",
  "gene_name": "Clusterin"
}